{
  "term_id": "UNKNOWN:0002",
  "gene_name": "Spermatogenesis-associated serine-rich protein 2",
  "gene": "UniProtKB:Q86XZ4",
  "term_label": "Unknown biological process",
  "gene_symbol": "SPATS2"
}